holo-[acyl-carrier-protein] biosynthetic process [GO:0031108] (biological process) Also known as: holo-[acyl-carrier protein] biosynthesis, holo-[acyl-carrier-protein] anabolism, holo-[acyl-carrier-protein] biosynthesis, holo-[acyl-carrier-protein] formation, holo-[acyl-carrier-protein] synthesis Relationships: is a type of macromolecule biosynthetic process [GO:0009059]; is a type of protein metabolic process [GO:0019538] Definition: The chemical reactions and pathways resulting in the formation of holo-[acyl-carrier protein]. Sources: GOC:mlg